{
  "term_id": "GO:0008083",
  "term_label": "growth factor activity",
  "gene_symbol": "IL11",
  "gene_name": "Interleukin-11",
  "gene": "UniProtKB:P20809"
}